{
  "term_label": "cytoplasm",
  "gene_symbol": "AIRIM",
  "gene_name": "AFG2-interacting ribosome maturation factor",
  "gene": "UniProtKB:Q9NX04",
  "term_id": "GO:0005737"
}